{
  "term_label": "Unknown cellular component",
  "gene_name": "E3 ubiquitin-protein ligase LRSAM1",
  "gene_symbol": "LRSAM1",
  "gene": "UniProtKB:Q6UWE0",
  "term_id": "UNKNOWN:0003"
}